{
  "gene_name": "Retinol-binding protein 1",
  "term_label": "fatty acid transport",
  "gene_symbol": "RBP1",
  "gene": "UniProtKB:P09455",
  "term_id": "GO:0015908"
}